regulation of cell-cell adhesion [GO:0022407] (biological process) Definition: Any process that modulates the frequency, rate or extent of attachment of a cell to another cell. Sources: GOC:isa_complete Relationships: is a type of regulation of cell adhesion [GO:0030155]; regulates cell-cell adhesion [GO:0098609] Subtypes: GO:0022408, positive regulation of cell-cell adhesion [GO:0022409], regulation of border follicle cell delamination [GO:0030710], GO:0033632, GO:0034110, regulation of heterotypic cell-cell adhesion [GO:0034114], regulation of calcium-dependent cell-cell adhesion [GO:0046586], GO:0051040, regulation of flocculation [GO:0060256], regulation of cell-cell adhesion involved in gastrulation [GO:0070587], regulation of pre-tubular aggregate formation by cell-cell signaling [GO:0072043], regulation of synaptic membrane adhesion [GO:0099179], GO:1903037, regulation of homophilic cell adhesion [GO:1903385], regulation of epithelial cell-cell adhesion involved in epithelium migration [GO:1903681], regulation of cell-cell adhesion mediated by cadherin [GO:2000047]